protein prenyltransferase activity [GO:0008318] (molecular function) Definition: Catalysis of the covalent addition of an isoprenoid group such as a farnesyl or geranylgeranyl group via thioether linkages to a cysteine residue in a protein. Sources: GOC:mah Relationships: is a type of prenyltransferase activity [GO:0004659]; is a type of catalytic activity, acting on a protein [GO:0140096] Subtypes: GO:0004660, protein geranylgeranyltransferase activity [GO:0004661]